{
  "term_id": "GO:0048237",
  "gene_name": "Alpha-2-macroglobulin receptor-associated protein",
  "term_label": "rough endoplasmic reticulum lumen",
  "gene_symbol": "LRPAP1",
  "gene": "UniProtKB:P30533"
}